{
  "term_id": "UNKNOWN:0002",
  "gene_symbol": "UBL3",
  "gene_name": "Ubiquitin-like protein 3",
  "term_label": "Unknown biological process",
  "gene": "UniProtKB:O95164"
}